{
  "term_id": "UNKNOWN:0003",
  "gene_name": "Putative uncharacterized protein OBSCN-AS1",
  "gene": "UniProtKB:Q96MR7",
  "gene_symbol": "OBSCN-AS1",
  "term_label": "Unknown cellular component"
}